{
  "gene_name": "Cathepsin F",
  "term_id": "GO:0051603",
  "term_label": "proteolysis involved in protein catabolic process",
  "gene_symbol": "CTSF",
  "gene": "UniProtKB:Q9UBX1"
}